{
  "term_id": "GO:0005615",
  "gene": "UniProtKB:Q86XP6",
  "term_label": "extracellular space",
  "gene_symbol": "GKN2",
  "gene_name": "Gastrokine-2"
}